{
  "term_id": "UNKNOWN:0001",
  "term_label": "Unknown molecular function",
  "gene_symbol": "PRKCSH",
  "gene_name": "Glucosidase 2 subunit beta",
  "gene": "UniProtKB:P14314"
}